positive regulation of asymmetric cell division [GO:0045770] (biological process) Relationships: is a type of regulation of asymmetric cell division [GO:0009786]; is a type of positive regulation of cell division [GO:0051781]; positively regulates asymmetric cell division [GO:0008356] Definition: Any process that activates or increases the frequency, rate or extent of asymmetric cell division. Also known as: up regulation of asymmetric cell division, up-regulation of asymmetric cell division, upregulation of asymmetric cell division, activation of asymmetric cell division, stimulation of asymmetric cell division Subtypes: positive regulation of male germ-line stem cell asymmetric division [GO:1904840] Sources: GOC:go_curators